{
  "gene_name": "E3 ubiquitin-protein ligase RNF213",
  "term_label": "cytosol",
  "gene_symbol": "RNF213",
  "term_id": "GO:0005829",
  "gene": "UniProtKB:Q63HN8"
}